{
  "term_id": "UNKNOWN:0003",
  "gene_symbol": "ZNF253",
  "gene_name": "Zinc finger protein 253",
  "gene": "UniProtKB:O75346",
  "term_label": "Unknown cellular component"
}